{
  "term_id": "GO:0005634",
  "gene": "UniProtKB:Q6B0I6",
  "term_label": "nucleus",
  "gene_name": "Lysine-specific demethylase 4D",
  "gene_symbol": "KDM4D"
}